heparan sulfate N-acetylglucosaminyltransferase activity [GO:0042328] (molecular function) Relationships: is a type of GO:0008375 Also known as: heparan sulphate N-acetylglucosaminyltransferase activity, heparin N-acetylglucosaminyltransferase activity Sources: GOC:ma Definition: Catalysis of the reaction: UDP-N-acetyl-D-glucosamine + heparan sulfate = UDP + (N-acetyl-D-glucosaminyl)-heparan sulfate.